{
  "term_label": "Unknown cellular component",
  "gene_name": "Glycine receptor subunit alpha-3",
  "gene_symbol": "GLRA3",
  "gene": "UniProtKB:O75311",
  "term_id": "UNKNOWN:0003"
}